{
  "gene_name": "Semaphorin-4G",
  "term_id": "GO:0071526",
  "gene": "UniProtKB:Q9NTN9",
  "term_label": "semaphorin-plexin signaling pathway",
  "gene_symbol": "SEMA4G"
}